{
  "gene_symbol": "NUDT19",
  "term_id": "UNKNOWN:0003",
  "gene": "UniProtKB:A8MXV4",
  "gene_name": "Acyl-coenzyme A diphosphatase NUDT19",
  "term_label": "Unknown cellular component"
}